system process [GO:0003008] (BP) Regulation: regulated by regulation of system process [GO:0044057] Sources: GOC:mtg_cardio Definition: A multicellular organismal process carried out by any of the organs or tissues in an organ system. An organ system is a regularly interacting or interdependent group of organs or tissues that work together to carry out a biological objective. Subtypes: GO:0003012, circulatory system process [GO:0003013], renal system process [GO:0003014], GO:0003016, GO:0007588, GO:0022600, nervous system process [GO:0050877], endocrine process [GO:0050886], hepaticobiliary system process [GO:0061007] Relationships: is a type of multicellular organismal process [GO:0032501] Also known as: organ system process